{
  "gene_name": "Putative ciliary rootlet coiled-coil protein-like 2 protein",
  "gene_symbol": "CROCCP3",
  "term_label": "Unknown molecular function",
  "gene": "UniProtKB:Q8IVE0",
  "term_id": "UNKNOWN:0001"
}